{
  "gene": "UniProtKB:Q06265",
  "gene_symbol": "EXOSC9",
  "term_label": "nuclear polyadenylation-dependent rRNA catabolic process",
  "gene_name": "Exosome complex component RRP45",
  "term_id": "GO:0071035"
}